{
  "term_label": "nucleolus",
  "gene_name": "Double-stranded RNA-specific editase B2",
  "gene_symbol": "ADARB2",
  "gene": "UniProtKB:Q9NS39",
  "term_id": "GO:0005730"
}